{
  "gene_symbol": "ZIM2",
  "gene": "UniProtKB:Q9NZV7",
  "term_id": "UNKNOWN:0003",
  "gene_name": "Zinc finger imprinted 2",
  "term_label": "Unknown cellular component"
}